{
  "term_id": "GO:0005175",
  "gene_symbol": "SIVA1",
  "term_label": "CD27 receptor binding",
  "gene": "UniProtKB:O15304",
  "gene_name": "Apoptosis regulatory protein Siva"
}